{
  "gene_name": "CD44 antigen",
  "gene_symbol": "CD44",
  "gene": "UniProtKB:P16070",
  "term_label": "cell adhesion",
  "term_id": "GO:0007155"
}